cellular response to polyamine macromolecule [GO:1904584] (BP) Relationships: is a type of cellular response to nitrogen compound [GO:1901699]; is a type of response to polyamine macromolecule [GO:1904583] References: PMID:20805360 Sources: GOC:TermGenie, GO_REF:0000071 Definition: Any process that results in a change in state or activity of a cell (in terms of movement, secretion, enzyme production, gene expression, etc.) as a result of a polyamine macromolecule stimulus. Also known as: cellular response to polyamine, cellular response to polyamines